{
  "term_label": "Unknown molecular function",
  "gene_symbol": "SLC22A12",
  "gene_name": "Solute carrier family 22 member 12",
  "gene": "UniProtKB:Q96S37",
  "term_id": "UNKNOWN:0001"
}